positive regulation of hepatocyte differentiation [GO:0070368] (biological process) Definition: Any process that activates or increases the rate or extent of hepatocyte differentiation. Sources: GOC:mah, GOC:sl Relationships: is a type of positive regulation of epithelial cell differentiation [GO:0030858]; is a type of GO:0051240; is a type of regulation of hepatocyte differentiation [GO:0070366]; RO_0002213 hepatocyte differentiation [GO:0070365] Also known as: positive regulation of liver cell differentiation, up regulation of hepatocyte differentiation, up-regulation of hepatocyte differentiation, upregulation of hepatocyte differentiation, activation of hepatocyte differentiation, stimulation of hepatocyte differentiation